{
  "term_label": "late endosome membrane",
  "term_id": "GO:0031902",
  "gene": "UniProtKB:P01920",
  "gene_name": "HLA class II histocompatibility antigen, DQ beta 1 chain",
  "gene_symbol": "HLA-DQB1"
}